{
  "gene_symbol": "TRIM2",
  "term_label": "Unknown cellular component",
  "gene": "UniProtKB:Q9C040",
  "term_id": "UNKNOWN:0003",
  "gene_name": "Tripartite motif-containing protein 2"
}